{
  "gene": "UniProtKB:P30273",
  "term_id": "GO:0045087",
  "gene_name": "High affinity immunoglobulin epsilon receptor subunit gamma",
  "term_label": "innate immune response",
  "gene_symbol": "FCER1G"
}